{
  "term_id": "GO:0007186",
  "gene": "UniProtKB:Q8TDS7",
  "gene_symbol": "MRGPRD",
  "gene_name": "Mas-related G-protein coupled receptor member D",
  "term_label": "G protein-coupled receptor signaling pathway"
}